{
  "term_label": "Unknown cellular component",
  "gene_symbol": "ANKEF1",
  "gene_name": "Ankyrin repeat and EF-hand domain-containing protein 1",
  "gene": "UniProtKB:Q9NU02",
  "term_id": "UNKNOWN:0003"
}